{
  "term_label": "ubiquitin-dependent protein catabolic process",
  "gene": "UniProtKB:Q76N89",
  "term_id": "GO:0006511",
  "gene_symbol": "HECW1",
  "gene_name": "E3 ubiquitin-protein ligase HECW1"
}